{
  "gene_symbol": "SUGP1",
  "term_label": "RNA binding",
  "term_id": "GO:0003723",
  "gene_name": "SURP and G-patch domain-containing protein 1",
  "gene": "UniProtKB:Q8IWZ8"
}